{
  "term_label": "lysosomal transport",
  "gene": "UniProtKB:Q9UID3",
  "gene_symbol": "VPS51",
  "term_id": "GO:0007041",
  "gene_name": "Vacuolar protein sorting-associated protein 51 homolog"
}